{
  "gene_symbol": "CLCN7",
  "term_id": "GO:1902476",
  "gene": "UniProtKB:P51798",
  "term_label": "chloride transmembrane transport",
  "gene_name": "H(+)_Cl(-) exchange transporter 7"
}